positive regulation of B cell anergy [GO:0002672] (BP) Relationships: is a type of positive regulation of B cell tolerance induction [GO:0002663]; is a type of regulation of B cell anergy [GO:0002670]; is a type of positive regulation of lymphocyte anergy [GO:0002913]; positively regulates GO:0002515 Also known as: positive regulation of B lymphocyte anergy, positive regulation of B-cell anergy, positive regulation of B-lymphocyte anergy, up regulation of B cell anergy, up-regulation of B cell anergy, upregulation of B cell anergy, activation of B cell anergy, stimulation of B cell anergy Sources: GOC:add Definition: Any process that activates or increases the frequency, rate, or extent of B cell anergy. Subtypes: GO:0002916, positive regulation of peripheral B cell anergy [GO:0002919]